positive regulation of DNA amplification [GO:1904525] (biological process) Definition: Any process that activates or increases the frequency, rate or extent of DNA amplification. Also known as: up regulation of DNA amplification, up-regulation of DNA amplification, upregulation of DNA amplification, activation of DNA amplification References: PMID:26195783 Sources: GOC:TermGenie, GO_REF:0000058 Relationships: is a type of GO:1904523; is a type of positive regulation of DNA biosynthetic process [GO:2000573]; positively regulates DNA amplification [GO:0006277]